negative regulation of plant organ morphogenesis [GO:1905422] (biological process) Definition: Any process that stops, prevents or reduces the frequency, rate or extent of plant organ morphogenesis. Sources: GOC:TermGenie, GOC:tb, GO_REF:0000058 Also known as: down regulation of plant organ morphogenesis, down-regulation of plant organ morphogenesis, downregulation of plant organ morphogenesis, inhibition of plant organ morphogenesis Relationships: is a type of negative regulation of developmental process [GO:0051093]; is a type of negative regulation of multicellular organismal process [GO:0051241]; is_a regulation of plant organ morphogenesis [GO:1905421]; negatively regulates plant organ morphogenesis [GO:1905392]